{
  "gene_name": "PHD and RING finger domain-containing protein 1",
  "gene": "UniProtKB:Q9P1Y6",
  "term_label": "Unknown cellular component",
  "term_id": "UNKNOWN:0003",
  "gene_symbol": "PHRF1"
}